regulation of endothelial cell-matrix adhesion [GO:1904904] (biological process) Relationships: is a type of regulation of cell-matrix adhesion [GO:0001952]; regulates endothelial cell-matrix adhesion [GO:0090673] References: PMID:19460962 Sources: GOC:BHF, GOC:BHF_miRNA, GOC:TermGenie, GOC:bc, GO_REF:0000058 Subtypes: GO:1904905, GO:1904906 Definition: Any process that modulates the frequency, rate or extent of endothelial cell-matrix adhesion.